violaxanthin de-epoxidase activity [GO:0046422] (molecular function) Relationships: is a type of GO:0120546 Definition: Catalysis of the reaction: violaxanthin + 2 ascorbate = zeaxanthin + 2 dehydroascorbate + 2 H2O; and antheraxanthin + ascorbate = zeaxanthin + dehydroascorbate + H2O. Also known as: VDE, violaxanthin:ascorbate oxidoreductase activity Sources: EC:1.23.5.1, GOC:ai, ISBN:0471331309